{
  "term_id": "GO:0060070",
  "gene_symbol": "FRZB",
  "term_label": "canonical Wnt signaling pathway",
  "gene_name": "Secreted frizzled-related protein 3",
  "gene": "UniProtKB:Q92765"
}